{
  "gene_name": "Programmed cell death protein 5",
  "term_label": "nucleus",
  "gene_symbol": "PDCD5",
  "gene": "UniProtKB:O14737",
  "term_id": "GO:0005634"
}